{
  "term_label": "plasma membrane",
  "gene_symbol": "OR51T1",
  "gene": "UniProtKB:Q8NGJ9",
  "gene_name": "Olfactory receptor 51T1",
  "term_id": "GO:0005886"
}